{
  "term_label": "cell migration",
  "gene_name": "Rho-related GTP-binding protein RhoF",
  "gene": "UniProtKB:Q9HBH0",
  "gene_symbol": "RHOF",
  "term_id": "GO:0016477"
}